{
  "term_id": "GO:0004659",
  "gene": "UniProtKB:Q86YH6",
  "term_label": "prenyltransferase activity",
  "gene_name": "All trans-polyprenyl-diphosphate synthase PDSS2",
  "gene_symbol": "PDSS2"
}